{
  "term_id": "GO:0050830",
  "gene_name": "Guanylate-binding protein 7",
  "gene_symbol": "GBP7",
  "term_label": "defense response to Gram-positive bacterium",
  "gene": "UniProtKB:Q8N8V2"
}